{
  "gene": "UniProtKB:P25025",
  "term_label": "C-C chemokine binding",
  "gene_symbol": "CXCR2",
  "gene_name": "C-X-C chemokine receptor type 2",
  "term_id": "GO:0019957"
}